{
  "gene_symbol": "IRAK2",
  "gene_name": "Interleukin-1 receptor-associated kinase-like 2",
  "term_label": "cytoplasm",
  "term_id": "GO:0005737",
  "gene": "UniProtKB:O43187"
}